{
  "term_label": "Unknown biological process",
  "gene_symbol": "UNC79",
  "gene": "UniProtKB:Q9P2D8",
  "term_id": "UNKNOWN:0002",
  "gene_name": "Protein unc-79 homolog"
}